{
  "gene_symbol": "UNQ6126_PRO20091",
  "term_label": "Unknown molecular function",
  "gene": "UniProtKB:Q6UXV3",
  "gene_name": "Uncharacterized protein UNQ6126_PRO20091",
  "term_id": "UNKNOWN:0001"
}